{
  "term_label": "peptidyl-proline 4-dioxygenase activity",
  "gene": "UniProtKB:Q9GZT9",
  "gene_symbol": "EGLN1",
  "gene_name": "Egl nine homolog 1",
  "term_id": "GO:0031545"
}